{
  "term_label": "metalloendopeptidase activity",
  "gene_name": "Endothelin-converting enzyme-like 1",
  "gene": "UniProtKB:O95672",
  "gene_symbol": "ECEL1",
  "term_id": "GO:0004222"
}